galactose 1-dehydrogenase (NADP+) activity [GO:0047910] (molecular function) Relationships: is a type of oxidoreductase activity, acting on the CH-OH group of donors, NAD or NADP as acceptor [GO:0016616] Definition: Catalysis of the reaction: D-galactose + NADP+ = D-galactonolactone + NADPH. Sources: EC:1.1.1.120, MetaCyc:GALACTOSE-1-DEHYDROGENASE-NADP+-RXN Also known as: D-galactose dehydrogenase (NADP+), D-galactose:NADP+ 1-oxidoreductase activity